response to estradiol [GO:0032355] (biological process) Relationships: is a type of GO:0033993; is a type of response to oxygen-containing compound [GO:1901700] Also known as: response to E2 stimulus, response to estradiol stimulus Subtypes: GO:0071392 Sources: GOC:mah, ISBN:0911910123 Definition: Any process that results in a change in state or activity of a cell or an organism (in terms of movement, secretion, enzyme production, gene expression, etc.) as a result of stimulus by estradiol, a C18 steroid hormone hydroxylated at C3 and C17 that acts as a potent estrogen.